{
  "gene_symbol": "NCOA4",
  "gene_name": "Nuclear receptor coactivator 4",
  "term_label": "response to hormone",
  "term_id": "GO:0009725",
  "gene": "UniProtKB:Q13772"
}